{
  "term_label": "nucleus",
  "gene_name": "Zinc finger protein 547",
  "gene_symbol": "ZNF547",
  "term_id": "GO:0005634",
  "gene": "UniProtKB:Q8IVP9"
}